{
  "term_label": "DNA-directed DNA polymerase activity",
  "gene": "UniProtKB:Q9HCU8",
  "gene_symbol": "POLD4",
  "gene_name": "DNA polymerase delta subunit 4",
  "term_id": "GO:0003887"
}